{
  "gene": "UniProtKB:A6NES4",
  "term_id": "UNKNOWN:0002",
  "term_label": "Unknown biological process",
  "gene_name": "Maestro heat-like repeat-containing protein family member 2A",
  "gene_symbol": "MROH2A"
}